{
  "gene_symbol": "KRTAP4-4",
  "term_id": "GO:0042633",
  "term_label": "hair cycle",
  "gene_name": "Keratin-associated protein 4-4",
  "gene": "UniProtKB:Q9BYR3"
}